{
  "gene": "UniProtKB:Q96JJ3",
  "gene_symbol": "ELMO2",
  "term_id": "UNKNOWN:0003",
  "term_label": "Unknown cellular component",
  "gene_name": "Engulfment and cell motility protein 2"
}